{
  "gene_name": "Tuberin",
  "term_id": "GO:0051726",
  "gene": "UniProtKB:P49815",
  "term_label": "regulation of cell cycle",
  "gene_symbol": "TSC2"
}